{
  "gene_symbol": "KNSTRN",
  "term_id": "GO:0007051",
  "gene_name": "Small kinetochore-associated protein",
  "term_label": "spindle organization",
  "gene": "UniProtKB:Q9Y448"
}